{
  "gene_symbol": "EMP2",
  "gene_name": "Epithelial membrane protein 2",
  "term_label": "regulation of cell-matrix adhesion",
  "term_id": "GO:0001952",
  "gene": "UniProtKB:P54851"
}